histone H4K5ac reader activity [GO:0140012] (molecular function) Note: Note that the residue position corresponds to the canonical human H4 histone (UniProtKB:P02309); this residue is conserved across all eukaryotes. Note that the initiation methionine is cleaved, so the first residue is S1. References: PMID:18406326, PMID:20709061 Also known as: H4K5ac modified histone binding Definition: A histone reader that recognizes a histone H4 acetylated at lysine 5. Relationships: is a type of histone H4 reader activity [GO:0140008]